{
  "gene": "UniProtKB:O94901",
  "term_id": "GO:0034993",
  "gene_name": "SUN domain-containing protein 1",
  "gene_symbol": "SUN1",
  "term_label": "meiotic nuclear membrane microtubule tethering complex"
}